{
  "gene_symbol": "RCC2",
  "gene": "UniProtKB:Q9P258",
  "term_id": "GO:0051987",
  "term_label": "positive regulation of attachment of spindle microtubules to kinetochore",
  "gene_name": "Protein RCC2"
}